{
  "term_label": "Unknown biological process",
  "gene_symbol": "DYRK2",
  "term_id": "UNKNOWN:0002",
  "gene_name": "Dual specificity tyrosine-phosphorylation-regulated kinase 2",
  "gene": "UniProtKB:Q92630"
}